{
  "gene": "UniProtKB:O60346",
  "gene_name": "PH domain leucine-rich repeat-containing protein phosphatase 1",
  "term_id": "GO:0005737",
  "term_label": "cytoplasm",
  "gene_symbol": "PHLPP1"
}